{
  "gene_name": "Transportin-1",
  "term_id": "GO:0008139",
  "gene": "UniProtKB:Q92973",
  "term_label": "nuclear localization sequence binding",
  "gene_symbol": "TNPO1"
}